{
  "gene_name": "N-acylneuraminate cytidylyltransferase",
  "gene": "UniProtKB:Q8NFW8",
  "gene_symbol": "CMAS",
  "term_label": "Unknown cellular component",
  "term_id": "UNKNOWN:0003"
}